regulation of meiotic spindle elongation [GO:1902119] (biological process) References: PMID:23370392 Sources: GOC:TermGenie Relationships: is a type of regulation of spindle elongation [GO:0032887]; is a type of regulation of reproductive process [GO:2000241]; RO_0002211 meiotic spindle elongation [GO:0051232] Subtypes: GO:1902120 Definition: Any process that modulates the frequency, rate or extent of meiotic spindle elongation. Also known as: regulation of spindle elongation during meiosis